RNA polymerase II transcription repressor complex [GO:0090571] (cellular component) Subtypes: negative cofactor 2 complex [GO:0017054], DRM complex [GO:0070176], Mad-Max-mSin3A complex [GO:0070439], GO:0070440, Mad-Max complex [GO:0070443], Tle3-Aes complex [GO:0070722], Cyc8(Ssn6)-Tup1 general repressor complex [GO:0160051], beta-catenin-ICAT complex [GO:1990711] Sources: GOC:tb Relationships: is a type of transcription repressor complex [GO:0017053]; is a type of nuclear protein-containing complex [GO:0140513] Definition: A protein complex, located in the nucleus, that possesses activity that prevents or downregulates transcription from a RNA polymerase II promoter.